monensin A catabolic process [GO:1901729] (biological process) Also known as: monensin A breakdown, monensin A catabolism, monensin A degradation, monensin breakdown, monensin catabolism, monensin degradation Relationships: is a type of alcohol catabolic process [GO:0046164]; is a type of carboxylic acid catabolic process [GO:0046395] Sources: GOC:TermGenie, GOC:yaf, UniPathway:UPA00178 Definition: The chemical reactions and pathways resulting in the breakdown of monensin A.